{
  "term_id": "UNKNOWN:0001",
  "gene_symbol": "TCP11L2",
  "gene_name": "T-complex protein 11-like protein 2",
  "term_label": "Unknown molecular function",
  "gene": "UniProtKB:Q8N4U5"
}